{
  "gene": "UniProtKB:Q9HC23",
  "gene_symbol": "PROK2",
  "term_label": "endothelial cell proliferation",
  "term_id": "GO:0001935",
  "gene_name": "Prokineticin-2"
}